{
  "term_id": "GO:0005634",
  "gene": "UniProtKB:O75179",
  "gene_name": "Ankyrin repeat domain-containing protein 17",
  "term_label": "nucleus",
  "gene_symbol": "ANKRD17"
}